behavioral defense response to nematode [GO:0002212] (biological process) Definition: A behavioral response seeking to protect an organism from an a perceived external threat from a nematode or nematodes to that organism. Relationships: is a type of behavioral defense response [GO:0002209]; is a type of defense response to nematode [GO:0002215] References: PMID:14506883 Sources: GOC:add Also known as: behavioural defense response to nematode